{
  "gene_name": "1-acylglycerol-3-phosphate O-acyltransferase ABHD5",
  "gene_symbol": "ABHD5",
  "gene": "UniProtKB:Q8WTS1",
  "term_label": "lysophosphatidic acid acyltransferase activity",
  "term_id": "GO:0042171"
}